{
  "term_id": "GO:0005886",
  "gene_symbol": "TRBV6-4",
  "gene_name": "T cell receptor beta variable 6-4",
  "term_label": "plasma membrane",
  "gene": "UniProtKB:A0A1B0GX49"
}